{
  "term_label": "immune response",
  "gene_name": "Interleukin-20",
  "gene_symbol": "IL20",
  "gene": "UniProtKB:Q9NYY1",
  "term_id": "GO:0006955"
}